megasporocyte differentiation [GO:1904159] (biological process) Definition: The process in which a relatively unspecialized cell acquires the specialized features of a megasporocyte. Sources: GOC:TermGenie, GOC:tair_curators, GO_REF:0000086 Also known as: megaspore mother cell differentiation Note: The process aimed at the progression of a megasporocyte cell over time, from initial commitment of the cell to a specific fate, to the fully functional differentiated cell. A megasporocyte is a diploid (2n) cell that undergoes meiosis and forms four haploid (1n) megaspores; also called megaspore mother cell. Relationships: is a type of sporocyte differentiation [GO:0048533]